1-phosphatidyl-1D-myo-inositol 3,5-bisphosphate catabolic process [GO:1903101] (biological process) Relationships: is a type of GO:0031161; is a type of 1-phosphatidyl-1D-myo-inositol 3,5-bisphosphate metabolic process [GO:1903100] References: PMID:19037259 Sources: GOC:TermGenie, GOC:bhm, GO_REF:0000068 Also known as: 1-phosphatidyl-1D-myo-inositol 3,5-bisphosphate breakdown, 1-phosphatidyl-1D-myo-inositol 3,5-bisphosphate catabolism, 1-phosphatidyl-1D-myo-inositol 3,5-bisphosphate degradation Definition: The chemical reactions and pathways resulting in the breakdown of 1-phosphatidyl-1D-myo-inositol 3,5-bisphosphate.